{
  "term_id": "GO:0005634",
  "gene_symbol": "TOB1",
  "gene_name": "Protein Tob1",
  "term_label": "nucleus",
  "gene": "UniProtKB:P50616"
}